Ubp3-Bre5 deubiquitination complex [GO:1990861] (CC) References: PMID:12778054, PMID:18391941 Sources: GOC:rb Relationships: is a type of peptidase complex [GO:1905368] Also known as: Ubp3-Bre5 ubiquitin protease complex Definition: A protein complex that cleaves ubiquitin from specific substrates. In the budding yeast Saccharomyces cerevisiae, this complex consists of Ubp3p and Bre5p.